{
  "term_id": "GO:0015182",
  "term_label": "L-asparagine transmembrane transporter activity",
  "gene": "UniProtKB:Q9NVC3",
  "gene_name": "Sodium-coupled neutral amino acid transporter 7",
  "gene_symbol": "SLC38A7"
}